cerebral cortex GABAergic interneuron differentiation [GO:0021892] (biological process) Definition: The process in which a relatively unspecialized cell acquires specialized features of a GABAergic interneuron residing in the cerebral cortex. Relationships: is a type of cerebral cortex neuron differentiation [GO:0021895]; is a type of GABAergic neuron differentiation [GO:0097154] References: PMID:12626695 Sources: GOC:cls, GOC:dgh, GOC:dph, GOC:jid, GO_REF:0000021